N-acetylneuraminate 4-O-acetyltransferase activity [GO:0047185] (molecular function) Definition: Catalysis of the reaction: N-acetylneuraminate + acetyl-CoA = N-acetyl-4-O-acetylneuraminate + CoA. Sources: EC:2.3.1.44, RHEA:18305 Also known as: sialate O-acetyltransferase, acetyl-CoA:N-acetylneuraminate 4-O-acetyltransferase activity Relationships: is a type of O-acetyltransferase activity [GO:0016413]